multicellular organismal process [GO:0032501] (biological process) Definition: Any biological process, occurring at the level of a multicellular organism, pertinent to its function. Note: Note that this term is in the subset of terms that should not be used for direct gene product annotation. Instead, select a child term or, if no appropriate child term exists, please request a new term. Direct annotations to this term may be amended during annotation QC. Subtypes: ossification [GO:0001503], morphogenesis of a branching structure [GO:0001763], cell activation [GO:0001775], cytokine production [GO:0001816], production of molecular mediator involved in inflammatory response [GO:0002532], system process [GO:0003008], circadian regulation of heart rate [GO:0003053], multicellular organism development [GO:0007275], pattern specification process [GO:0007389], GO:0007585, digestion [GO:0007586], GO:0007610, GO:0008340, GO:0009561, post-embryonic development [GO:0009791], seed germination [GO:0009845], pollen germination [GO:0009846], meristem determinacy [GO:0010022], GO:0010073, seed dormancy process [GO:0010162], muscle attachment [GO:0016203], stem cell population maintenance [GO:0019827], midbrain-hindbrain boundary maturation during brain development [GO:0022004], midbrain-hindbrain boundary maturation during neural plate development [GO:0022005], GO:0022404, multicellular organism adhesion [GO:0022608], sleep [GO:0030431], pseudocleavage [GO:0030588], GO:0031424, neurotrophin production [GO:0032898], secretion by tissue [GO:0032941], multicellular organismal response to stress [GO:0033555], plasma lipoprotein particle clearance [GO:0034381], pupariation [GO:0035073], pupation [GO:0035074], GO:0035264, organ growth [GO:0035265], scab formation [GO:0035314], otolith tethering [GO:0035889], molting cycle [GO:0042303], GO:0043480, multi-multicellular organism process [GO:0044706], transcytosis [GO:0045056], photoreceptor cell maintenance [GO:0045494], polyphenic determination [GO:0048647], tissue remodeling [GO:0048771], multicellular organismal-level homeostasis [GO:0048871], coagulation [GO:0050817], multicellular organismal movement [GO:0050879], GO:0055046, GO:0055127, innervation [GO:0060384], organism emergence from protective structure [GO:0071684], plasma lipoprotein particle organization [GO:0071827], GO:0080189, GO:0090130, response to high population density [GO:0090664], bud dormancy process [GO:0097207], amyloid-beta clearance [GO:0097242], acquisition of seed longevity [GO:0140547], callus formation [GO:1990110] Also known as: organismal physiological process, single-multicellular organism process Sources: GOC:curators, GOC:dph, GOC:isa_complete, GOC:tb Regulation: regulated by GO:0051239; positively regulated by positive regulation of multicellular organismal process [GO:0051240]; negatively regulated by negative regulation of multicellular organismal process [GO:0051241] Relationships: is a type of biological_process [GO:0008150]